negative regulation of sphingolipid mediated signaling pathway [GO:1902069] (biological process) Also known as: down regulation of sphingolipid mediated signaling pathway, down-regulation of sphingolipid mediated signaling pathway, downregulation of sphingolipid mediated signaling pathway, inhibition of sphingolipid mediated signaling pathway, down regulation of sphingolipid signaling pathway, down-regulation of sphingolipid signaling pathway, downregulation of sphingolipid signaling pathway, inhibition of sphingolipid signaling pathway, negative regulation of sphingolipid signaling pathway Definition: Any process that stops, prevents or reduces the frequency, rate or extent of sphingolipid signaling. References: PMID:20870412 Sources: GOC:TermGenie Relationships: is_a negative regulation of signal transduction [GO:0009968]; is a type of GO:1902068; negatively regulates sphingolipid mediated signaling pathway [GO:0090520]